{
  "gene_name": "Probable ATP-dependent RNA helicase DHX40",
  "term_id": "GO:0034458",
  "term_label": "3'-5' RNA helicase activity",
  "gene": "UniProtKB:Q8IX18",
  "gene_symbol": "DHX40"
}